{
  "gene_name": "Exocyst complex component 1",
  "term_label": "phosphatidylinositol-4,5-bisphosphate binding",
  "term_id": "GO:0005546",
  "gene": "UniProtKB:Q9NV70",
  "gene_symbol": "EXOC1"
}